{
  "term_id": "GO:0000724",
  "term_label": "double-strand break repair via homologous recombination",
  "gene_name": "Structural maintenance of chromosomes protein 6",
  "gene_symbol": "SMC6",
  "gene": "UniProtKB:Q96SB8"
}